phenanthrene catabolic process [GO:0042216] (biological process) Definition: The chemical reactions and pathways resulting in the breakdown of phenanthrene, a tricyclic aromatic hydrocarbon. Sources: GOC:jl Also known as: phenanthrene breakdown, phenanthrene catabolism, phenanthrene degradation Relationships: is a type of GO:0042178; is a type of hydrocarbon catabolic process [GO:0120253] Subtypes: GO:0018956, GO:0018957